L-serine-phosphatidylethanolamine phosphatidyltransferase activity [GO:0106245] (molecular function) Definition: Catalysis of the reaction: L-1-phosphatidylethanolamine + L-serine = L-1-phosphatidylserine + ethanolamine. Relationships: is a type of phosphotransferase activity, for other substituted phosphate groups [GO:0016780] References: PMID:19014349, PMID:31869331 Sources: RHEA:27606